{
  "term_id": "GO:0005739",
  "gene": "UniProtKB:P22033",
  "gene_name": "Methylmalonyl-CoA mutase, mitochondrial",
  "term_label": "mitochondrion",
  "gene_symbol": "MMUT"
}